{
  "gene_symbol": "TMEM59L",
  "term_id": "UNKNOWN:0001",
  "term_label": "Unknown molecular function",
  "gene": "UniProtKB:Q9UK28",
  "gene_name": "Transmembrane protein 59-like"
}